{
  "term_label": "cell differentiation",
  "gene_name": "Homeobox protein Nkx-2.6",
  "gene_symbol": "NKX2-6",
  "term_id": "GO:0030154",
  "gene": "UniProtKB:A6NCS4"
}